{
  "term_label": "nucleus",
  "gene": "UniProtKB:Q5VVQ6",
  "term_id": "GO:0005634",
  "gene_symbol": "YOD1",
  "gene_name": "Ubiquitin thioesterase OTU1"
}